{
  "gene_symbol": "PHETA2",
  "gene": "UniProtKB:Q6ICB4",
  "term_label": "early endosome",
  "term_id": "GO:0005769",
  "gene_name": "Sesquipedalian-2"
}